GlcNAc(2)-PP-Dol mannosyltransferase activity [GO:0120562] (molecular function) Sources: GOC:curators Subtypes: GDP-Man:Man(3)GlcNAc(2)-PP-Dol alpha-1,2-mannosyltransferase activity [GO:0004377], GDP-Man:Man(1)GlcNAc(2)-PP-Dol alpha-1,3-mannosyltransferase activity [GO:0004378], chitobiosyldiphosphodolichol beta-mannosyltransferase activity [GO:0004578], dol-P-Man:Man(7)GlcNAc(2)-PP-Dol alpha-1,6-mannosyltransferase activity [GO:0052917], GO:0052918, dol-P-Man:Man(5)GlcNAc(2)-PP-Dol alpha-1,3-mannosyltransferase activity [GO:0052925], dol-P-Man:Man(6)GlcNAc(2)-PP-Dol alpha-1,2-mannosyltransferase activity [GO:0052926], GDP-Man:Man(2)GlcNAc(2)-PP-Dol alpha-1,6-mannosyltransferase activity [GO:0102704] Relationships: is a type of mannosyltransferase activity [GO:0000030] Definition: Catalysis of the transfer of a mannosyl residue to GlcNAc(2)-PP-Dol bearing 0-8 mannoses during synthesis of the N-glycan precursor.